{
  "gene_symbol": "RBMY1E",
  "gene": "UniProtKB:A6NEQ0",
  "gene_name": "RNA-binding motif protein, Y chromosome, family 1 member E",
  "term_label": "mRNA splicing, via spliceosome",
  "term_id": "GO:0000398"
}